{
  "term_id": "UNKNOWN:0002",
  "gene_name": "Uncharacterized protein C5orf46",
  "term_label": "Unknown biological process",
  "gene": "UniProtKB:Q6UWT4",
  "gene_symbol": "C5orf46"
}